{
  "gene_symbol": "SH2D5",
  "gene": "UniProtKB:Q6ZV89",
  "term_id": "UNKNOWN:0001",
  "gene_name": "SH2 domain-containing protein 5",
  "term_label": "Unknown molecular function"
}